{
  "term_id": "GO:0090200",
  "gene": "UniProtKB:Q96A26",
  "gene_name": "Protein FAM162A",
  "term_label": "positive regulation of release of cytochrome c from mitochondria",
  "gene_symbol": "FAM162A"
}